{
  "gene_symbol": "TRIM71",
  "gene_name": "E3 ubiquitin-protein ligase TRIM71",
  "term_label": "post-transcriptional regulation of gene expression",
  "term_id": "GO:0010608",
  "gene": "UniProtKB:Q2Q1W2"
}